{
  "gene": "UniProtKB:Q99616",
  "term_id": "GO:0048245",
  "gene_symbol": "CCL13",
  "term_label": "eosinophil chemotaxis",
  "gene_name": "C-C motif chemokine 13"
}